{
  "term_label": "plasma membrane",
  "term_id": "GO:0005886",
  "gene": "UniProtKB:Q8NG85",
  "gene_name": "Olfactory receptor 2L3",
  "gene_symbol": "OR2L3"
}